{
  "term_id": "GO:0004966",
  "gene_symbol": "GALR1",
  "gene": "UniProtKB:P47211",
  "gene_name": "Galanin receptor type 1",
  "term_label": "galanin receptor activity"
}